{
  "term_label": "guanyl-nucleotide exchange factor activity",
  "term_id": "GO:0005085",
  "gene_symbol": "RGL3",
  "gene": "UniProtKB:Q3MIN7",
  "gene_name": "Ral guanine nucleotide dissociation stimulator-like 3"
}